{
  "gene": "UniProtKB:P02810",
  "term_id": "UNKNOWN:0003",
  "term_label": "Unknown cellular component",
  "gene_name": "Salivary acidic proline-rich phosphoprotein 1_2",
  "gene_symbol": "PRH2"
}